positive regulation of receptor recycling [GO:0001921] (biological process) Definition: Any process that activates or increases the frequency, rate or extent of receptor recycling. Also known as: up regulation of receptor recycling, up-regulation of receptor recycling, upregulation of receptor recycling, activation of receptor recycling, stimulation of receptor recycling Relationships: is a type of regulation of receptor recycling [GO:0001919]; is a type of GO:0010604; is_a positive regulation of signaling [GO:0023056]; positively regulates receptor recycling [GO:0001881] Sources: GOC:add